{
  "gene_name": "Beta-1,3-galactosyltransferase 9",
  "gene": "UniProtKB:A8MXE2",
  "term_label": "Unknown biological process",
  "term_id": "UNKNOWN:0002",
  "gene_symbol": "B3GALT9"
}